{
  "gene_symbol": "KRT36",
  "gene_name": "Keratin, type I cuticular Ha6",
  "term_label": "intermediate filament organization",
  "gene": "UniProtKB:O76013",
  "term_id": "GO:0045109"
}